medulla reticulospinal tract morphogenesis [GO:0021976] (BP) Definition: Generation of a long process of a CNS neuron, that carries efferent (outgoing) action potentials from the cell body in the medulla towards target cells in the spinal cord. Sources: GOC:cls, GOC:dgh, GOC:dph, GOC:jid, GO_REF:0000021 Relationships: is_a GO:0021952